{
  "gene": "UniProtKB:Q86SG5",
  "gene_name": "Protein S100-A7A",
  "term_label": "calcium-dependent protein binding",
  "gene_symbol": "S100A7A",
  "term_id": "GO:0048306"
}